{
  "term_id": "GO:0006954",
  "gene": "UniProtKB:P21731",
  "term_label": "inflammatory response",
  "gene_symbol": "TBXA2R",
  "gene_name": "Thromboxane A2 receptor"
}